{
  "gene": "UniProtKB:P24821",
  "gene_name": "Tenascin",
  "gene_symbol": "TNC",
  "term_id": "UNKNOWN:0001",
  "term_label": "Unknown molecular function"
}